{
  "gene": "UniProtKB:Q15735",
  "gene_name": "Phosphatidylinositol 4,5-bisphosphate 5-phosphatase A",
  "term_id": "GO:0046030",
  "gene_symbol": "INPP5J",
  "term_label": "inositol trisphosphate phosphatase activity"
}